symbiont genome ejection through host cell envelope [GO:0039678] (biological process) Subtypes: symbiont genome ejection through host cell envelope, contractile tail mechanism [GO:0099000], symbiont genome ejection through host cell envelope, long flexible tail mechanism [GO:0099001], GO:0099002 Relationships: is a type of viral process [GO:0016032]; is part of symbiont entry into host cell [GO:0046718] Also known as: phage genome ejection, viral genome injection through bacterial membranes, viral genome ejection through host cell envelope References: PMID:23385786, PMID:31663016 Sources: GOC:ch, VZ:986 Definition: Entry of a symbiont's genome into the host cell through the host cell envelope. Occurs in non-enveloped prokaryotic viruses. Caudovirales carry an ejection apparatus that can be long and contractile, long and noncontractile, or short, and is able to penetrate the host cell envelope to deliver the viral genome into the host cell cytoplasm.